{
  "gene": "UniProtKB:P17081",
  "term_id": "GO:0003924",
  "term_label": "GTPase activity",
  "gene_symbol": "RHOQ",
  "gene_name": "Rho-related GTP-binding protein RhoQ"
}